{
  "gene_name": "RNA-binding protein 47",
  "term_label": "Unknown biological process",
  "gene": "UniProtKB:A0AV96",
  "term_id": "UNKNOWN:0002",
  "gene_symbol": "RBM47"
}